{
  "gene_name": "Eukaryotic translation initiation factor 3 subunit C",
  "term_label": "translation initiation factor activity",
  "gene_symbol": "EIF3C",
  "gene": "UniProtKB:Q99613",
  "term_id": "GO:0003743"
}